{
  "gene_symbol": "MASP1",
  "term_id": "GO:0005615",
  "gene": "UniProtKB:P48740",
  "gene_name": "Mannan-binding lectin serine protease 1",
  "term_label": "extracellular space"
}